{
  "term_id": "UNKNOWN:0001",
  "term_label": "Unknown molecular function",
  "gene": "UniProtKB:Q96CE8",
  "gene_symbol": "TM4SF18",
  "gene_name": "Transmembrane 4 L6 family member 18"
}